folic acid transmembrane transporter activity [GO:0008517] (molecular function) Subtypes: GO:0008518, folic acid:proton symporter activity [GO:0140211] Definition: Enables the transfer of folic acid (pteroylglutamic acid) from one side of a membrane to the other. Folic acid is widely distributed as a member of the vitamin B complex and is essential for the synthesis of purine and pyrimidines. Relationships: is_a amide transmembrane transporter activity [GO:0042887]; is a type of carboxylic acid transmembrane transporter activity [GO:0046943]; is a type of modified amino acid transmembrane transporter activity [GO:0072349]; is a type of vitamin transmembrane transporter activity [GO:0090482]; is part of folic acid transport [GO:0015884] Sources: GOC:ai Also known as: folate transmembrane transporter activity, folate transporter activity, vitamin B9 transporter activity, vitamin M transporter activity, folic acid transporter activity